{
  "gene_name": "Tumor necrosis factor receptor superfamily member EDAR",
  "term_label": "plasma membrane",
  "gene": "UniProtKB:Q9UNE0",
  "term_id": "GO:0005886",
  "gene_symbol": "EDAR"
}